{
  "gene": "UniProtKB:Q8WWL2",
  "gene_symbol": "SPIRE2",
  "gene_name": "Protein spire homolog 2",
  "term_label": "polar body extrusion after meiotic divisions",
  "term_id": "GO:0040038"
}